{
  "gene_name": "Cadherin EGF LAG seven-pass G-type receptor 3",
  "term_label": "Unknown molecular function",
  "gene": "UniProtKB:Q9NYQ7",
  "gene_symbol": "CELSR3",
  "term_id": "UNKNOWN:0001"
}